{
  "gene_symbol": "HR",
  "term_label": "regulation of transcription by RNA polymerase II",
  "gene_name": "Lysine-specific demethylase hairless",
  "term_id": "GO:0006357",
  "gene": "UniProtKB:O43593"
}